{
  "term_label": "Unknown molecular function",
  "term_id": "UNKNOWN:0001",
  "gene": "UniProtKB:Q15276",
  "gene_name": "Rab GTPase-binding effector protein 1",
  "gene_symbol": "RABEP1"
}